{
  "term_id": "GO:0005615",
  "gene": "UniProtKB:Q9H4G4",
  "gene_name": "Golgi-associated plant pathogenesis-related protein 1",
  "term_label": "extracellular space",
  "gene_symbol": "GLIPR2"
}